{
  "gene_name": "Putative UPF0607 protein LOC392364",
  "term_label": "Unknown biological process",
  "gene_symbol": "Q5PR19",
  "term_id": "UNKNOWN:0002",
  "gene": "UniProtKB:Q5PR19"
}